positive regulation of osteoblast differentiation [GO:0045669] (biological process) Sources: GOC:go_curators Definition: Any process that activates or increases the frequency, rate or extent of osteoblast differentiation. Relationships: is a type of positive regulation of cell differentiation [GO:0045597]; is a type of GO:0045667; positively regulates osteoblast differentiation [GO:0001649] Also known as: up regulation of osteoblast differentiation, up-regulation of osteoblast differentiation, upregulation of osteoblast differentiation, activation of osteoblast differentiation, stimulation of osteoblast differentiation